{
  "term_id": "GO:0016324",
  "gene_symbol": "SLC17A3",
  "gene_name": "Sodium-dependent phosphate transport protein 4",
  "gene": "UniProtKB:O00476",
  "term_label": "apical plasma membrane"
}